{
  "term_id": "GO:0004967",
  "gene_name": "Glucagon-like peptide 2 receptor",
  "term_label": "glucagon receptor activity",
  "gene": "UniProtKB:O95838",
  "gene_symbol": "GLP2R"
}